{
  "gene_name": "1-acyl-sn-glycerol-3-phosphate acyltransferase gamma",
  "term_label": "endoplasmic reticulum",
  "term_id": "GO:0005783",
  "gene": "UniProtKB:Q9NRZ7",
  "gene_symbol": "AGPAT3"
}